{
  "gene": "UniProtKB:Q96A35",
  "term_label": "translation",
  "term_id": "GO:0006412",
  "gene_name": "Large ribosomal subunit protein uL24m",
  "gene_symbol": "MRPL24"
}